{
  "gene": "UniProtKB:Q9HCC6",
  "gene_name": "Transcription factor HES-4",
  "term_label": "DNA-binding transcription factor activity, RNA polymerase II-specific",
  "gene_symbol": "HES4",
  "term_id": "GO:0000981"
}